{
  "gene_name": "Calmodulin-3",
  "term_label": "cytoplasm",
  "gene": "UniProtKB:P0DP25",
  "term_id": "GO:0005737",
  "gene_symbol": "CALM3"
}